{
  "gene_name": "NAD-dependent protein deacetylase sirtuin-1",
  "term_label": "nuclear inner membrane",
  "gene": "UniProtKB:Q96EB6",
  "gene_symbol": "SIRT1",
  "term_id": "GO:0005637"
}